plastid DNA replication [GO:0033259] (biological process) Also known as: replication of plastid DNA, plastid DNA synthesis Relationships: is a type of DNA-templated DNA replication [GO:0006261]; is_a GO:0033258; occurs in GO:0009536 Sources: GOC:mah Definition: The process in which new strands of DNA are synthesized in a plastid.